{
  "gene": "UniProtKB:Q9BXJ3",
  "term_id": "GO:0005615",
  "gene_symbol": "C1QTNF4",
  "gene_name": "Complement C1q tumor necrosis factor-related protein 4",
  "term_label": "extracellular space"
}